epigenetic programming in the zygotic pronuclei [GO:0044725] (biological process) Relationships: is a type of epigenetic programming of gene expression [GO:0043045] Subtypes: epigenetic programing of female pronucleus [GO:0044726], GO:0044727, epigenetic programming in the endosperm [GO:0141044] References: PMID:22868271 Sources: GOC:sp Also known as: chromatin reprogramming in the zygote Definition: The global programming of epigenetic modifications in the zygote following fertilization. The paternal genome undergoes active DNA demethylation before the first cell division, while the adjacent maternal genome is protected from this process.